regulation of (+)-kotanin biosynthetic process [GO:1900692] (biological process) Definition: Any process that modulates the frequency, rate or extent of (+)-kotanin biosynthetic process. Sources: GOC:TermGenie, GOC:di Also known as: regulation of (+)-kotanin anabolism, regulation of (+)-kotanin biosynthesis, regulation of (+)-kotanin formation, regulation of (+)-kotanin synthesis Relationships: is a type of GO:1900376; regulates (+)-kotanin biosynthetic process [GO:1900596] Subtypes: negative regulation of (+)-kotanin biosynthetic process [GO:1900693], GO:1900694